venom-mediated blood coagulation [GO:0044469] (biological process) Sources: GOC:jl Also known as: envenomation promoting blood coagulation, envenomation resulting in positive regulation of blood coagulation in another organism, envenomation resulting in positive regulation of blood coagulation in other organism Subtypes: venom-mediated platelet aggregation [GO:0044478] Definition: A process in which an organism initiates, promotes, or enhances blood coagulation in another organism via the action of a venom. Relationships: is a type of venom-mediated perturbation of blood coagulation [GO:0044468]